{
  "term_label": "plasma membrane",
  "gene": "UniProtKB:Q8NGE2",
  "term_id": "GO:0005886",
  "gene_symbol": "OR2AP1",
  "gene_name": "Olfactory receptor 2AP1"
}